{
  "gene": "UniProtKB:Q9UHM6",
  "gene_symbol": "OPN4",
  "term_id": "GO:0071482",
  "gene_name": "Melanopsin",
  "term_label": "cellular response to light stimulus"
}